cellular response to cycloalkane [GO:0071408] (biological process) Definition: Any process that results in a change in state or activity of a cell (in terms of movement, secretion, enzyme production, gene expression, etc.) as a result of a cycloalkane stimulus. A cycloalkane is a cyclic saturated hydrocarbon having the general formula CnH2n. Relationships: is a type of GO:0014071; is a type of cellular response to chemical stimulus [GO:0070887] Sources: GOC:mah